DEAD/H-box RNA helicase binding [GO:0017151] (molecular function) Sources: GOC:jl Relationships: is a type of enzyme binding [GO:0019899] Definition: Binding to a DEAD/H-box RNA helicase.